mRNA methyltransferase activity [GO:0008174] (molecular function) Relationships: is a type of RNA methyltransferase activity [GO:0008173]; is a type of S-adenosylmethionine-dependent methyltransferase activity [GO:0008757] Subtypes: mRNA m(6)A methyltransferase activity [GO:0001734], GO:0004482, mRNA (2'-O-methyladenosine-N6-)-methyltransferase activity [GO:0016422], mRNA (adenine-N1-)-methyltransferase activity [GO:0061953], mRNA (cytidine-5-)-methyltransferase activity [GO:0062152], internal mRNA (guanine-N7-)-methyltransferase activity [GO:0160090] Definition: Catalysis of the transfer of a methyl group from S-adenosyl-L-methionine to a nucleoside residue in an mRNA molecule. Sources: GOC:mah